bacterial-type RNA polymerase core enzyme binding [GO:0001000] (molecular function) Also known as: eubacterial-type RNA polymerase core enzyme binding Sources: GOC:txnOH Note: Should omega be included here? Subtypes: GO:0001052 Definition: Binding to a bacterial-type RNA polymerase core enzyme, typically consisting of two alpha, one beta, one beta prime, and one omega subunit. Relationships: is a type of RNA polymerase core enzyme binding [GO:0043175]